{
  "term_id": "GO:0005634",
  "gene_symbol": "ZNF773",
  "gene": "UniProtKB:Q6PK81",
  "term_label": "nucleus",
  "gene_name": "Zinc finger protein 773"
}